{
  "gene_symbol": "KLHL18",
  "term_id": "GO:1990756",
  "term_label": "ubiquitin-like ligase-substrate adaptor activity",
  "gene": "UniProtKB:O94889",
  "gene_name": "Kelch-like protein 18"
}